{
  "term_id": "GO:0016460",
  "gene_name": "Myosin-1",
  "term_label": "myosin II complex",
  "gene": "UniProtKB:P12882",
  "gene_symbol": "MYH1"
}